cobalamin catabolic process [GO:0042366] (biological process) Definition: The chemical reactions and pathways resulting in the breakdown of cobalamin (vitamin B12), a water-soluble vitamin characterized by possession of a corrin nucleus containing a cobalt atom. Also known as: cobalamin breakdown, cobalamin catabolism, cobalamin degradation, vitamin B12 catabolic process, vitamin B12 catabolism Relationships: is a type of cobalamin metabolic process [GO:0009235]; is a type of GO:0033015; is a type of water-soluble vitamin catabolic process [GO:0042365] Sources: GOC:go_curators